peripheral T cell tolerance induction [GO:0002458] (biological process) Sources: GOC:jal, ISBN:0781735149 Definition: Tolerance induction of T cells in the periphery, in this case, any location in the body other than the thymus. Subtypes: T cell tolerance induction in mucosal-associated lymphoid tissue [GO:0002403], T cell tolerance induction to tumor cell [GO:0002411] Regulation: regulated by regulation of peripheral T cell tolerance induction [GO:0002849]; negatively regulated by GO:0002850; positively regulated by GO:0002851 Also known as: peripheral T lymphocyte tolerance induction, peripheral T-cell tolerance induction, peripheral T-lymphocyte tolerance induction Relationships: is a type of T cell mediated immunity [GO:0002456]; is_a peripheral tolerance induction [GO:0002465]; is a type of GO:0002517